3-phenylpropionate dioxygenase complex [GO:0009334] (cellular component) References: PMID:9603882 Sources: GOC:jl, MetaCyc:HCAMULTI-CPLX Relationships: is_a oxidoreductase complex [GO:1990204] Note: See also the molecular function term '3-phenylpropionate dioxygenase activity ; GO:0008695'. Definition: Enzyme complex consisting of four proteins: the two subunits of the hydroxylase component (hcaE and hcaF), a ferredoxin (hcaC) and a ferredoxin reductase (hcaD). Converts 3-phenylpropionic acid (PP) into cis-3-(3-carboxyethyl)-3,5-cyclohexadiene-1,2-diol (PP-dihydrodiol).